D-valine catabolic process [GO:1902079] (biological process) Also known as: D-valine breakdown, D-valine catabolism, D-valine degradation Relationships: is_a branched-chain amino acid catabolic process [GO:0009083]; is_a D-amino acid catabolic process [GO:0019478]; is a type of GO:1902114 Definition: The chemical reactions and pathways resulting in the breakdown of D-valine. References: PMID:23085840 Sources: GOC:TermGenie